{
  "gene": "UniProtKB:Q16348",
  "gene_symbol": "SLC15A2",
  "term_label": "dipeptide transmembrane transporter activity",
  "gene_name": "Solute carrier family 15 member 2",
  "term_id": "GO:0071916"
}